{
  "term_id": "UNKNOWN:0002",
  "gene": "UniProtKB:Q8N377",
  "gene_symbol": "Q8N377",
  "gene_name": "Putative uncharacterized protein LOC387726",
  "term_label": "Unknown biological process"
}